{
  "gene": "UniProtKB:O15315",
  "gene_symbol": "RAD51B",
  "term_id": "GO:0000724",
  "gene_name": "DNA repair protein RAD51 homolog 2",
  "term_label": "double-strand break repair via homologous recombination"
}